{
  "term_id": "GO:0060122",
  "gene_name": "Harmonin",
  "gene_symbol": "USH1C",
  "term_label": "inner ear receptor cell stereocilium organization",
  "gene": "UniProtKB:Q9Y6N9"
}